{
  "gene_name": "Phosphoprotein associated with glycosphingolipid-enriched microdomains 1",
  "gene_symbol": "PAG1",
  "term_label": "intracellular signal transduction",
  "term_id": "GO:0035556",
  "gene": "UniProtKB:Q9NWQ8"
}